positive regulation of mesenchymal cell apoptotic process involved in metanephric nephron morphogenesis [GO:0072306] (biological process) Definition: Any process that increases the occurrence or rate of mesenchymal stem cell death by apoptotic process that contributes to the shaping of the nephron in the metanephros. Sources: GOC:mtg_apoptosis, GOC:mtg_kidney_jan10 Relationships: is a type of GO:0072041; is a type of regulation of mesenchymal cell apoptotic process involved in metanephric nephron morphogenesis [GO:0072304]; is a type of positive regulation of mesenchymal cell apoptotic process involved in metanephros development [GO:1900213]; RO_0002213 GO:0072309; positively regulates mesenchymal cell apoptotic process involved in metanephric nephron morphogenesis [GO:1901147] Also known as: positive regulation of mesenchymal stem cell apoptotic process involved in metanephric nephron morphogenesis, positive regulation of mesenchymal stem cell apoptosis involved in metanephric nephron morphogenesis